{
  "gene_name": "E3 ubiquitin-protein ligase TRIM39",
  "term_label": "negative regulation of proteasomal ubiquitin-dependent protein catabolic process",
  "gene": "UniProtKB:Q9HCM9",
  "term_id": "GO:0032435",
  "gene_symbol": "TRIM39"
}